{
  "gene": "UniProtKB:O94886",
  "gene_name": "CSC1-like protein 1",
  "gene_symbol": "TMEM63A",
  "term_label": "plasma membrane",
  "term_id": "GO:0005886"
}